{
  "term_label": "plasma membrane",
  "gene_symbol": "GPR160",
  "gene": "UniProtKB:Q9UJ42",
  "gene_name": "Probable G-protein coupled receptor 160",
  "term_id": "GO:0005886"
}